hedgehog receptor activity [GO:0008158] (MF) Also known as: patched activity Definition: Combining with a member of the hedgehog protein family and transmitting the signal across the membrane to initiate a change in cell activity. Relationships: is a type of GO:0004888; has part hedgehog family protein binding [GO:0097108] References: PMID:9278137 Sources: GOC:bf, GOC:go_curators